{
  "term_id": "GO:0042383",
  "gene_symbol": "RYR1",
  "term_label": "sarcolemma",
  "gene_name": "Ryanodine receptor 1",
  "gene": "UniProtKB:P21817"
}